{
  "gene": "UniProtKB:Q9H7C4",
  "gene_symbol": "SYNC",
  "term_id": "GO:0042383",
  "gene_name": "Syncoilin",
  "term_label": "sarcolemma"
}